{
  "gene": "UniProtKB:P02708",
  "term_id": "GO:0005886",
  "gene_name": "Acetylcholine receptor subunit alpha",
  "term_label": "plasma membrane",
  "gene_symbol": "CHRNA1"
}